regulation of haustorium mother cell formation [GO:0075193] (biological process) Definition: Any process that modulates the frequency, rate or extent of symbiont haustorium mother cell formation. The host is defined as the larger of the organisms involved in a symbiotic interaction. Subtypes: GO:0075194, negative regulation of haustorium mother cell formation [GO:0075195] Sources: GOC:pamgo_curators Note: Note that this term should not be used to annotate gene products of the host. It should only be used to annotate those gene products from the symbiont involved in this process. Relationships: is_a regulation of developmental process [GO:0050793]; regulates haustorium mother cell formation [GO:0075192] Also known as: regulation of haustorium mother cell formation on or near host